negative regulation of nitrogen utilization [GO:0045847] (biological process) Relationships: is a type of regulation of nitrogen utilization [GO:0006808]; is a type of negative regulation of response to nutrient levels [GO:0032108]; negatively regulates GO:0019740 Also known as: down regulation of nitrogen utilization, down-regulation of nitrogen utilization, downregulation of nitrogen utilization, inhibition of nitrogen utilization Sources: GOC:go_curators Definition: Any process that stops, prevents, or reduces the frequency, rate or extent of nitrogen utilization. Subtypes: negative regulation of ammonia assimilation cycle [GO:2001249]